positive regulation of synaptic vesicle recycling [GO:1903423] (biological process) Definition: Any process that activates or increases the frequency, rate or extent of synaptic vesicle recycling. References: PMID:22745285 Sources: GOC:PARL, GOC:TermGenie, GOC:pad, GO_REF:0000058 Also known as: up regulation of synaptic vesicle recycling, up-regulation of synaptic vesicle recycling, upregulation of synaptic vesicle recycling, activation of kiss-and-run synaptic vesicle recycling, activation of kiss-and-stay synaptic vesicle recycling, activation of synaptic vesicle recycling, positive regulation of kiss-and-run synaptic vesicle recycling, positive regulation of kiss-and-stay synaptic vesicle recycling, up regulation of kiss-and-run synaptic vesicle recycling, up regulation of kiss-and-stay synaptic vesicle recycling, up-regulation of kiss-and-run synaptic vesicle recycling, up-regulation of kiss-and-stay synaptic vesicle recycling, upregulation of kiss-and-run synaptic vesicle recycling, upregulation of kiss-and-stay synaptic vesicle recycling Note: An example of this is mouse LRRK2 (Q5S006) in PMID:21307259 inferred from mutant phenotype Relationships: is a type of positive regulation of transport [GO:0051050]; is a type of GO:1903421; positively regulates synaptic vesicle recycling [GO:0036465] Subtypes: positive regulation of synaptic vesicle endocytosis [GO:1900244]